{
  "term_label": "G protein-coupled receptor kinase activity",
  "gene_name": "Beta-adrenergic receptor kinase 2",
  "gene": "UniProtKB:P35626",
  "term_id": "GO:0004703",
  "gene_symbol": "GRK3"
}